{
  "term_id": "UNKNOWN:0002",
  "gene_name": "Calmodulin regulator protein PCP4",
  "gene_symbol": "PCP4",
  "gene": "UniProtKB:P48539",
  "term_label": "Unknown biological process"
}